cuticle pattern formation [GO:0035017] (biological process) Subtypes: adult chitin-based cuticle pattern formation [GO:0035018], GO:0035293 Definition: The regionalization process that gives rise to the patterns of cell differentiation in the cuticle. Sources: GOC:bf Relationships: is a type of GO:0003002; is part of cuticle development [GO:0042335]